{
  "gene": "UniProtKB:A6NKF1",
  "gene_symbol": "SAC3D1",
  "term_id": "GO:0051298",
  "term_label": "centrosome duplication",
  "gene_name": "SAC3 domain-containing protein 1"
}